myosin light chain binding [GO:0032027] (molecular function) Definition: Binding to a light chain of a myosin complex. Sources: GOC:mah Relationships: is a type of myosin binding [GO:0017022] Subtypes: GO:0032030, myosin II light chain binding [GO:0032033], myosin VI light chain binding [GO:0070856]